{
  "term_label": "DNA-binding transcription repressor activity, RNA polymerase II-specific",
  "term_id": "GO:0001227",
  "gene_name": "Zinc finger CCCH domain-containing protein 8",
  "gene_symbol": "ZC3H8",
  "gene": "UniProtKB:Q8N5P1"
}